{
  "gene_symbol": "NTM",
  "gene": "UniProtKB:Q9P121",
  "term_id": "GO:0048787",
  "term_label": "presynaptic active zone membrane",
  "gene_name": "Neurotrimin"
}